{
  "term_label": "regulation of transcription by RNA polymerase II",
  "gene_symbol": "ZNF787",
  "gene_name": "Zinc finger protein 787",
  "term_id": "GO:0006357",
  "gene": "UniProtKB:Q6DD87"
}